{
  "term_label": "regulation of mitotic nuclear division",
  "gene_symbol": "CDCA2",
  "gene_name": "Cell division cycle-associated protein 2",
  "term_id": "GO:0007088",
  "gene": "UniProtKB:Q69YH5"
}